{
  "gene": "UniProtKB:Q24JP5",
  "term_label": "positive regulation of Wnt signaling pathway",
  "term_id": "GO:0030177",
  "gene_name": "Transmembrane protein 132A",
  "gene_symbol": "TMEM132A"
}